{
  "gene_name": "Lysophospholipid acyltransferase 2",
  "gene_symbol": "MBOAT2",
  "term_id": "GO:0016020",
  "term_label": "membrane",
  "gene": "UniProtKB:Q6ZWT7"
}